hexachlorocyclohexane metabolic process [GO:0019497] (biological process) Also known as: hexachlorocyclohexane metabolism Definition: The chemical reactions and pathways involving hexachlorocyclohexane, a cyclohexane derivative with 6 chlorine atoms attached to the hexane ring. Hexachlorocyclohexane consists of a mixture of 8 different isomers and was used a commercial insecticide. It is persistent in the environment, causing serious soil pollution. Sources: UM-BBD_pathwayID:ghch, UM-BBD_pathwayID:hch Relationships: is a type of halogenated hydrocarbon metabolic process [GO:0042197] Subtypes: beta-1,2,3,4,5,6-hexachlorocyclohexane metabolic process [GO:0018877], GO:0018919